{
  "gene_name": "Coiled-coil domain-containing protein 13",
  "gene_symbol": "CCDC13",
  "gene": "UniProtKB:Q8IYE1",
  "term_label": "cytoplasmic microtubule organization",
  "term_id": "GO:0031122"
}